{
  "term_id": "GO:0005615",
  "gene_name": "C-X-C motif chemokine 6",
  "term_label": "extracellular space",
  "gene_symbol": "CXCL6",
  "gene": "UniProtKB:P80162"
}